N-terminal protein amino acid carboxylation [GO:0050989] (biological process) Relationships: is a type of N-terminal protein amino acid modification [GO:0031365] Definition: The carboxylation of the N-terminal amino acid of proteins. Sources: GOC:ai